{
  "gene_symbol": "TUBA1A",
  "term_id": "GO:0005737",
  "term_label": "cytoplasm",
  "gene": "UniProtKB:Q71U36",
  "gene_name": "Tubulin alpha-1A chain"
}